{
  "term_label": "cytosol",
  "gene": "UniProtKB:P00326",
  "term_id": "GO:0005829",
  "gene_symbol": "ADH1C",
  "gene_name": "Alcohol dehydrogenase 1C"
}